aldonic acid catabolic process [GO:0046176] (biological process) Sources: ISBN:0198506732 Relationships: is a type of GO:0072329 Definition: The chemical reactions and pathways resulting in the breakdown of aldonic acid, a monocarboxylic acid with a chain of three or more carbon atoms, derived from an aldose by oxidation of the aldehydic group. Also known as: aldonic acid breakdown, aldonic acid catabolism, aldonic acid degradation Subtypes: galactonate catabolic process [GO:0019584], GO:0046181, L-idonate catabolic process [GO:0046183]